histone H2B reader activity [GO:0140071] (molecular function) Relationships: is a type of histone reader activity [GO:0140566] References: PMID:11498575, PMID:25688442, PMID:31082667, PMID:34726351 Definition: A histone reader that specifically binds either to an unmodified histone H2B or a form modified by a post-translational modification on a specific residue. The most common PTMs on histones are methylation, acetylation and phosphorylation. Also known as: histone H2B reader